3,8-divinyl protochlorophyllide a 8-vinyl-reductase (NADPH) activity [GO:0033728] (molecular function) Sources: EC:1.3.1.75 Also known as: 3,8-divinyl protochlorophyllide a 8-vinyl reductase activity, 3,8-divinyl protochlorophyllide a 8-vinyl-reductase (NADPH) activit, 4VCR, [4-vinyl]chlorophyllide a reductase activity, chlorophyllide-a:NADP+ oxidoreductase activity Definition: Catalysis of the reaction: protochlorophyllide a + NADP+ = 3,8-divinyl protochlorophyllide a + NADPH + H+, and chlorophyllide a + NADP+ = 3,8-divinyl chlorophyllide a + NADPH + H+. Relationships: is a type of oxidoreductase activity, acting on the CH-CH group of donors, NAD or NADP as acceptor [GO:0016628]